{
  "term_label": "nucleus",
  "gene_name": "Methyl-CpG-binding domain protein 3",
  "gene": "UniProtKB:O95983",
  "term_id": "GO:0005634",
  "gene_symbol": "MBD3"
}